{
  "term_id": "GO:0005769",
  "gene": "UniProtKB:Q9BZZ2",
  "term_label": "early endosome",
  "gene_name": "Sialoadhesin",
  "gene_symbol": "SIGLEC1"
}